{
  "gene_symbol": "ITGB7",
  "gene_name": "Integrin beta-7",
  "gene": "UniProtKB:P26010",
  "term_id": "GO:0007229",
  "term_label": "integrin-mediated signaling pathway"
}